{
  "gene_name": "Serine_threonine-protein phosphatase with EF-hands 2",
  "gene": "UniProtKB:O14830",
  "gene_symbol": "PPEF2",
  "term_id": "GO:0005634",
  "term_label": "nucleus"
}